{
  "gene": "UniProtKB:Q4VCS5",
  "term_label": "bicellular tight junction",
  "gene_name": "Angiomotin",
  "gene_symbol": "AMOT",
  "term_id": "GO:0005923"
}